{
  "term_label": "Unknown cellular component",
  "gene": "UniProtKB:A6NGB7",
  "gene_symbol": "TMEM221",
  "term_id": "UNKNOWN:0003",
  "gene_name": "Transmembrane protein 221"
}